{
  "gene": "UniProtKB:P11166",
  "term_id": "GO:0005886",
  "gene_name": "Solute carrier family 2, facilitated glucose transporter member 1",
  "term_label": "plasma membrane",
  "gene_symbol": "SLC2A1"
}